{
  "term_id": "UNKNOWN:0003",
  "term_label": "Unknown cellular component",
  "gene": "UniProtKB:Q8WXF7",
  "gene_name": "Atlastin-1",
  "gene_symbol": "ATL1"
}